{
  "gene_symbol": "RAB3IP",
  "term_id": "GO:0005829",
  "gene": "UniProtKB:Q96QF0",
  "term_label": "cytosol",
  "gene_name": "Rab-3A-interacting protein"
}